{
  "gene_symbol": "PDE3A",
  "gene_name": "cGMP-inhibited 3',5'-cyclic phosphodiesterase 3A",
  "term_label": "cytosol",
  "gene": "UniProtKB:Q14432",
  "term_id": "GO:0005829"
}